positive regulation of Wnt-Frizzled-LRP5/6 complex assembly [GO:1904712] (biological process) Definition: Any process that activates or increases the frequency, rate or extent of Wnt-Frizzled-LRP5/6 complex assembly. Sources: GOC:PARL, GOC:TermGenie, GOC:bf, GO_REF:0000058 Also known as: positive regulation of Wnt-FZD-LRP5/6 trimeric complex assembly, positive regulation of Wnt-FZD-LRP5/6 trimeric complex formation, up regulation of Frizzled-LRP5/6 complex assembly, up regulation of Wnt-FZD-LRP5/6 trimeric complex assembly, up regulation of Wnt-FZD-LRP5/6 trimeric complex formation, up-regulation of Frizzled-LRP5/6 complex assembly, up-regulation of Wnt-FZD-LRP5/6 trimeric complex assembly, up-regulation of Wnt-FZD-LRP5/6 trimeric complex formation, upregulation of Frizzled-LRP5/6 complex assembly, upregulation of Wnt-FZD-LRP5/6 trimeric complex assembly, upregulation of Wnt-FZD-LRP5/6 trimeric complex formation, activation of Frizzled-LRP5/6 complex assembly, activation of WNT-FZD-LRP5 complex assembly, activation of WNT-FZD-LRP5 complex formation, activation of WNT-FZD-LRP6 complex assembly, activation of WNT-FZD-LRP6 complex formation, activation of Wnt-FZD-LRP5/6 trimeric complex assembly, activation of Wnt-FZD-LRP5/6 trimeric complex formation, positive regulation of WNT-FZD-LRP5 complex assembly, positive regulation of WNT-FZD-LRP5 complex formation, positive regulation of WNT-FZD-LRP6 complex assembly, positive regulation of WNT-FZD-LRP6 complex formation, up regulation of WNT-FZD-LRP5 complex assembly, up regulation of WNT-FZD-LRP5 complex formation, up regulation of WNT-FZD-LRP6 complex assembly, up regulation of WNT-FZD-LRP6 complex formation, up-regulation of WNT-FZD-LRP5 complex assembly, up-regulation of WNT-FZD-LRP5 complex formation, up-regulation of WNT-FZD-LRP6 complex assembly, up-regulation of WNT-FZD-LRP6 complex formation, upregulation of WNT-FZD-LRP5 complex assembly, upregulation of WNT-FZD-LRP5 complex formation, upregulation of WNT-FZD-LRP6 complex assembly, upregulation of WNT-FZD-LRP6 complex formation, activation of Frizzled-LRP5/6 complex formation, activation of Wnt-induced Frizzled-LRP5/6 complex assembly, activation of Wnt-induced Frizzled-LRP5/6 complex formation, positive regulation of Frizzled-LRP5/6 complex assembly, positive regulation of Frizzled-LRP5/6 complex formation, positive regulation of Wnt-induced Frizzled-LRP5/6 complex assembly, positive regulation of Wnt-induced Frizzled-LRP5/6 complex formation, up regulation of Frizzled-LRP5/6 complex formation, up regulation of Wnt-induced Frizzled-LRP5/6 complex assembly, up regulation of Wnt-induced Frizzled-LRP5/6 complex formation, up-regulation of Frizzled-LRP5/6 complex formation, up-regulation of Wnt-induced Frizzled-LRP5/6 complex assembly, up-regulation of Wnt-induced Frizzled-LRP5/6 complex formation, upregulation of Frizzled-LRP5/6 complex formation, upregulation of Wnt-induced Frizzled-LRP5/6 complex assembly, upregulation of Wnt-induced Frizzled-LRP5/6 complex formation Relationships: is a type of positive regulation of protein-containing complex assembly [GO:0031334]; is_a GO:1904711; positively regulates GO:1904701